{
  "gene_name": "Early growth response protein 4",
  "gene": "UniProtKB:Q05215",
  "gene_symbol": "EGR4",
  "term_label": "regulation of transcription by RNA polymerase II",
  "term_id": "GO:0006357"
}